{
  "gene_name": "Calcipressin-2",
  "term_id": "GO:0005737",
  "gene_symbol": "RCAN2",
  "term_label": "cytoplasm",
  "gene": "UniProtKB:Q14206"
}